{
  "gene_name": "Ferric-chelate reductase 1",
  "gene": "UniProtKB:Q6ZNA5",
  "gene_symbol": "FRRS1",
  "term_label": "oxidoreductase activity, acting on metal ions",
  "term_id": "GO:0016722"
}